{
  "gene_symbol": "FGF23",
  "gene_name": "Fibroblast growth factor 23",
  "term_label": "cytoplasm",
  "term_id": "GO:0005737",
  "gene": "UniProtKB:Q9GZV9"
}